amide biosynthetic process [GO:0043604] (BP) Definition: The chemical reactions and pathways resulting in the formation of an amide, any derivative of an oxoacid in which an acidic hydroxy group has been replaced by an amino or substituted amino group. Subtypes: urea cycle [GO:0000050], pyoverdine biosynthetic process [GO:0002049], bradykinin biosynthetic process [GO:0002936], sphingomyelin biosynthetic process [GO:0006686], glutathione biosynthetic process [GO:0006750], biotin biosynthetic process [GO:0009102], ureide biosynthetic process [GO:0010137], coenzyme A biosynthetic process [GO:0015937], GO:0015940, rhizobactin 1021 biosynthetic process [GO:0019289], allantoin biosynthetic process [GO:0019428], vibriobactin biosynthetic process [GO:0019537], melatonin biosynthetic process [GO:0030187], peptide antibiotic biosynthetic process [GO:0030651], GO:0031169, indoleacetic acid amide conjugate biosynthetic process [GO:0033475], GO:0035499, chrysobactin biosynthetic process [GO:0042858], achromobactin biosynthetic process [GO:0042861], novobiocin biosynthetic process [GO:0043642], N-acetylneuraminate biosynthetic process [GO:0046380], ceramide biosynthetic process [GO:0046513], folic acid biosynthetic process [GO:0046656], phytochelatin biosynthetic process [GO:0046938], depsipeptide biosynthetic process [GO:0050763], fatty acid primary amide biosynthetic process [GO:0062112], L-asparagine biosynthetic process [GO:0070981], pyrrolysine biosynthetic process [GO:0071524], acyl-CoA biosynthetic process [GO:0071616], lactam biosynthetic process [GO:0072339], spermidine hydroxycinnamate conjugate biosynthetic process [GO:0080088], GO:0140654, viridicatumtoxin biosynthetic process [GO:0140872], piperine biosynthetic process [GO:0160181], tensidol A biosynthetic process [GO:1900605], tensidol B biosynthetic process [GO:1900608], GO:1900805, ochratoxin A biosynthetic process [GO:1900818], GO:1901103, bacitracin A biosynthetic process [GO:1901124], leukotriene D4 biosynthetic process [GO:1901750], lincomycin biosynthetic process [GO:1901774], gliotoxin biosynthetic process [GO:2001310] Relationships: is a type of biosynthetic process [GO:0009058]; is a type of amide metabolic process [GO:0043603] Sources: GOC:curators